{
  "gene_symbol": "VPS33B",
  "gene_name": "Vacuolar protein sorting-associated protein 33B",
  "gene": "UniProtKB:Q9H267",
  "term_id": "GO:0016192",
  "term_label": "vesicle-mediated transport"
}